intermediate filament organization [GO:0045109] (biological process) Relationships: is a type of intermediate filament cytoskeleton organization [GO:0045104]; is a type of GO:0097435 Also known as: intermediate filament organisation Sources: GOC:ai Subtypes: intermediate filament bundle assembly [GO:0045110] Definition: Control of the spatial distribution of intermediate filaments; includes organizing filaments into meshworks, bundles, or other structures, as by cross-linking.